{
  "gene_symbol": "NR4A3",
  "gene_name": "Nuclear receptor subfamily 4 group A member 3",
  "term_id": "GO:0035259",
  "gene": "UniProtKB:Q92570",
  "term_label": "nuclear glucocorticoid receptor binding"
}